{
  "gene_name": "Transducin-like enhancer protein 6",
  "gene": "UniProtKB:Q9H808",
  "gene_symbol": "TLE6",
  "term_id": "GO:0090090",
  "term_label": "negative regulation of canonical Wnt signaling pathway"
}